calcium-dependent cell-cell adhesion [GO:0016339] (biological process) Regulation: RO_0002211 by regulation of calcium-dependent cell-cell adhesion [GO:0046586]; positively regulated by positive regulation of calcium-dependent cell-cell adhesion [GO:0046587]; negatively regulated by GO:0046588 Also known as: calcium-dependent cell adhesion molecule activity Relationships: is a type of cell-cell adhesion [GO:0098609] Sources: GOC:hb Definition: The attachment of one cell to another cell via adhesion molecules that require the presence of calcium for the interaction.